{
  "term_id": "GO:0001965",
  "gene_name": "G-protein-signaling modulator 1",
  "term_label": "G-protein alpha-subunit binding",
  "gene": "UniProtKB:Q86YR5",
  "gene_symbol": "GPSM1"
}